cloacal septation [GO:0060197] (biological process) Relationships: is a type of GO:0035239; is part of cloaca development [GO:0035844] Definition: The separation of the single opening of the digestive, urinary, and reproductive tracts, the cloaca, into multiple isolated openings during development. Sources: GOC:dph, GOC:st Also known as: cloaca septation